URM1 activating enzyme activity [GO:0042292] (molecular function) Sources: GOC:mah Relationships: is a type of ubiquitin-like modifier activating enzyme activity [GO:0008641] Definition: Catalysis of the activation of the small ubiquitin-related modifier URM1, through the formation of an ATP-dependent high-energy thiolester bond.